{
  "gene_symbol": "MOB1B",
  "gene_name": "MOB kinase activator 1B",
  "gene": "UniProtKB:Q7L9L4",
  "term_id": "GO:0005737",
  "term_label": "cytoplasm"
}